{
  "term_id": "GO:0016973",
  "term_label": "poly(A)+ mRNA export from nucleus",
  "gene": "UniProtKB:P0DQW0",
  "gene_symbol": "ZC3H11C",
  "gene_name": "Zinc finger CCCH domain-containing protein 11C"
}